G protein-coupled acetylcholine receptor signaling pathway [GO:0007213] (biological process) Definition: A G protein-coupled receptor signaling pathway initiated by a ligand binding to an acetylcholine receptor on the surface of a target cell, and ends with regulation of a downstream cellular process, e.g. transcription. Sources: GOC:mah, ISBN:0815316194 Also known as: G-protein coupled acetylcholine receptor signaling pathway, acetylcholine receptor signalling, muscarinic pathway, muscarinic acetylcholine receptor signaling pathway Relationships: is_a G protein-coupled receptor signaling pathway [GO:0007186]; is a type of acetylcholine receptor signaling pathway [GO:0095500]; has part GO:0016907 Subtypes: adenylate cyclase-inhibiting G protein-coupled acetylcholine receptor signaling pathway [GO:0007197], GO:0007207, G protein-coupled acetylcholine receptor signaling pathway involved in heart process [GO:0086093], GO:1904065